rhombomere 6 morphogenesis [GO:0021667] (biological process) Definition: The process in which the anatomical structure of rhombomere 6 is generated and organized. Rhombomeres are transverse segments of the developing rhombencephalon. Rhombomeres are lineage restricted, express different genes from one another, and adopt different developmental fates. Rhombomeres are numbered in an anterior to posterior order. Relationships: is a type of GO:0021593; BFO_0000050 rhombomere 6 development [GO:0021572] Sources: GOC:cls, GOC:curators, GOC:dgh, GOC:dph, GOC:jid